{
  "gene_name": "E3 SUMO-protein ligase RanBP2",
  "gene_symbol": "RANBP2",
  "gene": "UniProtKB:P49792",
  "term_id": "GO:0005643",
  "term_label": "nuclear pore"
}